{
  "gene_symbol": "EBAG9",
  "gene_name": "Receptor-binding cancer antigen expressed on SiSo cells",
  "gene": "UniProtKB:O00559",
  "term_id": "GO:0030141",
  "term_label": "secretory granule"
}